{
  "gene_name": "Transmembrane protein 40",
  "term_label": "Unknown biological process",
  "gene_symbol": "TMEM40",
  "term_id": "UNKNOWN:0002",
  "gene": "UniProtKB:Q8WWA1"
}